alpha9-beta1 integrin-ADAM8 complex [GO:0071133] (cellular component) Definition: A protein complex that consists of an alpha9-beta1 integrin complex bound to the transmembrane metallopeptidase ADAM8. References: PMID:16995821 Also known as: ITGA9-ITGB1-ADAM8 complex Relationships: is a type of plasma membrane protein complex [GO:0098797]